phospholipase C-activating dopamine receptor signaling pathway [GO:0060158] (biological process) References: PMID:12675914 Sources: GOC:dph, GOC:signaling, GOC:tb Relationships: is a type of phospholipase C-activating G protein-coupled receptor signaling pathway [GO:0007200]; is a type of G protein-coupled dopamine receptor signaling pathway [GO:0007212] Definition: A phospholipase C-activating receptor G protein-coupled receptor signaling pathway initiated by dopamine binding to its receptor on the surface of a target cell, and ending with the regulation of a downstream cellular process, e.g. transcription. Regulation: negatively regulated by negative regulation of phospholipase C-activating dopamine receptor signaling pathway [GO:0060162] Also known as: activation of phospholipase C activity by dopamine receptor signaling pathway, activation of phospholipase C activity by dopamine receptor signalling pathway, dopamine receptor, phospholipase C activating pathway